{
  "gene_name": "Transmembrane protein 100",
  "term_label": "Unknown molecular function",
  "gene": "UniProtKB:Q9NV29",
  "term_id": "UNKNOWN:0001",
  "gene_symbol": "TMEM100"
}